{
  "gene": "UniProtKB:Q96HL8",
  "term_label": "phosphatidylinositol binding",
  "term_id": "GO:0035091",
  "gene_symbol": "SH3YL1",
  "gene_name": "SH3 domain-containing YSC84-like protein 1"
}